endosome to pigment granule transport [GO:0043485] (biological process) Definition: The directed movement of substances from endosomes to pigment granules. Sources: GOC:jl Relationships: is a type of intracellular transport [GO:0046907]; is part of pigment granule maturation [GO:0048757] Subtypes: endosome to melanosome transport [GO:0035646]